{
  "gene_name": "Protein kinase C zeta type",
  "term_id": "GO:0032869",
  "gene_symbol": "PRKCZ",
  "term_label": "cellular response to insulin stimulus",
  "gene": "UniProtKB:Q05513"
}